{
  "gene_name": "Large ribosomal subunit protein mL44",
  "gene_symbol": "MRPL44",
  "term_label": "Unknown molecular function",
  "term_id": "UNKNOWN:0001",
  "gene": "UniProtKB:Q9H9J2"
}